{
  "gene_symbol": "IGFBP3",
  "gene": "UniProtKB:P17936",
  "term_label": "extracellular space",
  "term_id": "GO:0005615",
  "gene_name": "Insulin-like growth factor-binding protein 3"
}